{
  "term_label": "neuron projection",
  "term_id": "GO:0043005",
  "gene_symbol": "DLG1",
  "gene": "UniProtKB:Q12959",
  "gene_name": "Disks large homolog 1"
}